{
  "term_id": "UNKNOWN:0003",
  "gene_symbol": "TBPL2",
  "gene_name": "TATA box-binding protein-like 2",
  "term_label": "Unknown cellular component",
  "gene": "UniProtKB:Q6SJ96"
}